{
  "term_id": "GO:0005737",
  "term_label": "cytoplasm",
  "gene_name": "Protein BEX3",
  "gene_symbol": "BEX3",
  "gene": "UniProtKB:Q00994"
}